{
  "term_id": "GO:0000785",
  "gene_name": "Protein Mis18-alpha",
  "term_label": "chromatin",
  "gene_symbol": "MIS18A",
  "gene": "UniProtKB:Q9NYP9"
}